{
  "term_label": "regulation of TOR signaling",
  "gene_name": "Transmembrane protein 127",
  "gene_symbol": "TMEM127",
  "term_id": "GO:0032006",
  "gene": "UniProtKB:O75204"
}